{
  "gene_symbol": "VAV3",
  "gene_name": "Guanine nucleotide exchange factor VAV3",
  "term_label": "small GTPase-mediated signal transduction",
  "term_id": "GO:0007264",
  "gene": "UniProtKB:Q9UKW4"
}